{
  "term_id": "GO:0070059",
  "gene_name": "E3 ubiquitin-protein ligase RNF186",
  "term_label": "intrinsic apoptotic signaling pathway in response to endoplasmic reticulum stress",
  "gene_symbol": "RNF186",
  "gene": "UniProtKB:Q9NXI6"
}